{
  "gene_symbol": "TIGD1",
  "term_id": "GO:0005634",
  "gene_name": "Tigger transposable element-derived protein 1",
  "gene": "UniProtKB:Q96MW7",
  "term_label": "nucleus"
}